{
  "term_id": "GO:0004674",
  "gene_name": "Serine_threonine-protein kinase WNK3",
  "gene": "UniProtKB:Q9BYP7",
  "gene_symbol": "WNK3",
  "term_label": "protein serine/threonine kinase activity"
}